{
  "gene_name": "Epithelial membrane protein 2",
  "term_id": "GO:2001046",
  "gene_symbol": "EMP2",
  "term_label": "positive regulation of integrin-mediated signaling pathway",
  "gene": "UniProtKB:P54851"
}